regulation of neurotransmitter receptor activity [GO:0099601] (biological process) Sources: GOC:dos Subtypes: regulation of NMDA receptor activity [GO:2000310], regulation of AMPA receptor activity [GO:2000311] Definition: Any process that modulates the frequency, rate or extent of neurotransmitter receptor activity. Modulation may be via an effect on ligand affinity, or effector function such as ion selectivity or pore opening/closing in ionotropic receptors. Relationships: is a type of regulation of signaling receptor activity [GO:0010469]; regulates neurotransmitter receptor activity [GO:0030594]